{
  "term_id": "GO:0007015",
  "gene_name": "Rho-related BTB domain-containing protein 2",
  "gene_symbol": "RHOBTB2",
  "gene": "UniProtKB:Q9BYZ6",
  "term_label": "actin filament organization"
}